{
  "term_label": "peroxisome",
  "gene": "UniProtKB:Q9BY49",
  "term_id": "GO:0005777",
  "gene_name": "Peroxisomal trans-2-enoyl-CoA reductase",
  "gene_symbol": "PECR"
}